{
  "gene": "UniProtKB:Q04864",
  "gene_symbol": "REL",
  "term_id": "GO:0045944",
  "gene_name": "Proto-oncogene c-Rel",
  "term_label": "positive regulation of transcription by RNA polymerase II"
}